{
  "term_label": "regulation of DNA-templated transcription",
  "term_id": "GO:0006355",
  "gene_symbol": "NFILZ",
  "gene": "UniProtKB:A0A5F9ZHS7",
  "gene_name": "NFIL3 like protein"
}